post-embryonic pelvic fin morphogenesis [GO:0035131] (biological process) Sources: GOC:dgh Relationships: is a type of post-embryonic appendage morphogenesis [GO:0035120]; is a type of pelvic fin morphogenesis [GO:0035139] Definition: The process, occurring after embryonic development, by which the anatomical structures of the pelvic fin are generated and organized. The pelvic fins are bilaterally paired fins mounted in a ventral-lateral position on most fish. These fins are used primarily for lateral mobility and propulsion.